{
  "term_label": "primary methylamine oxidase activity",
  "gene_symbol": "MAOB",
  "gene": "UniProtKB:P27338",
  "term_id": "GO:0008131",
  "gene_name": "Amine oxidase [flavin-containing] B"
}